{
  "term_id": "GO:0042500",
  "gene_name": "Signal peptide peptidase-like 3",
  "gene_symbol": "SPPL3",
  "term_label": "aspartic endopeptidase activity, intramembrane cleaving",
  "gene": "UniProtKB:Q8TCT6"
}